{
  "gene": "UniProtKB:O75334",
  "term_id": "GO:0050808",
  "gene_symbol": "PPFIA2",
  "term_label": "synapse organization",
  "gene_name": "Liprin-alpha-2"
}